{
  "term_label": "Unknown molecular function",
  "term_id": "UNKNOWN:0001",
  "gene": "UniProtKB:Q9Y6V7",
  "gene_name": "Probable ATP-dependent RNA helicase DDX49",
  "gene_symbol": "DDX49"
}